trans-synaptic signaling by neuropeptide [GO:0099540] (biological process) Definition: Cell-cell signaling between presynapse and postsynapse mediated by a peptide ligand crossing the synaptic cleft. Sources: GOC:dos Relationships: is a type of GO:0099537; is a type of synaptic signaling via neuropeptide [GO:0099538] Subtypes: retrograde trans-synaptic signaling by neuropeptide [GO:0099082], trans-synaptic signaling by neuropeptide, modulating synaptic transmission [GO:0099551]